{
  "gene_name": "Zinc finger protein 740",
  "gene_symbol": "ZNF740",
  "term_id": "GO:0003700",
  "gene": "UniProtKB:Q8NDX6",
  "term_label": "DNA-binding transcription factor activity"
}